{
  "term_label": "cell adhesion molecule binding",
  "gene": "UniProtKB:Q9Y5H7",
  "gene_symbol": "PCDHA5",
  "term_id": "GO:0050839",
  "gene_name": "Protocadherin alpha-5"
}